{
  "term_label": "Unknown biological process",
  "gene_name": "Uncharacterized protein",
  "gene": "UniProtKB:A0A6Q8PHA8",
  "term_id": "UNKNOWN:0002",
  "gene_symbol": "A0A6Q8PHA8"
}